{
  "term_id": "UNKNOWN:0002",
  "gene_name": "T cell receptor alpha joining 39 (Fragment)",
  "gene_symbol": "TRAJ39",
  "gene": "UniProtKB:A0A075B710",
  "term_label": "Unknown biological process"
}